{
  "gene_symbol": "NF2",
  "gene": "UniProtKB:P35240",
  "term_label": "apical part of cell",
  "gene_name": "Merlin",
  "term_id": "GO:0045177"
}